sno(s)RNA transcription [GO:0009302] (biological process) Relationships: is a type of GO:0006351; is a type of sno(s)RNA metabolic process [GO:0016074] Also known as: sRNA transcription, snoRNA transcription Definition: The synthesis of snoRNA class RNA (also referred to as sRNA in Archaea) from a DNA template. Subtypes: GO:0001014, snoRNA transcription by RNA polymerase II [GO:0001015] References: PMID:17284456 Sources: GOC:jl, GOC:krc